{
  "gene_name": "Calretinin",
  "term_label": "synapse",
  "gene": "UniProtKB:P22676",
  "term_id": "GO:0045202",
  "gene_symbol": "CALB2"
}